{
  "gene_name": "Contactin-associated protein-like 3B",
  "gene_symbol": "CNTNAP3B",
  "gene": "UniProtKB:Q96NU0",
  "term_label": "plasma membrane",
  "term_id": "GO:0005886"
}